carveol dehydrogenase activity [GO:0018459] (molecular function) Definition: Catalysis of the reaction: (1S,5R)-carveol + NADP+ = (R)-carvone + H+ + NADPH. Relationships: is a type of GO:0016616 Sources: EC:1.1.1.243, RHEA:13629 Also known as: (-)-trans-carveol dehydrogenase activity, (-)-trans-carveol:NADP+ oxidoreductase activity